carbon tetrachloride metabolic process [GO:0018885] (biological process) Also known as: carbon tetrachloride metabolism Sources: UM-BBD_pathwayID:ctc Relationships: is a type of halogenated hydrocarbon metabolic process [GO:0042197] Definition: The chemical reactions and pathways involving carbon tetrachloride, a toxic, carcinogenic compound which is used as a general solvent in industrial degreasing operations. It is also used as grain fumigant and a chemical intermediate in the production of refrigerants. Subtypes: anaerobic carbon tetrachloride metabolic process [GO:0018886], carbon tetrachloride catabolic process [GO:0019382]